{
  "term_id": "UNKNOWN:0003",
  "gene": "UniProtKB:S4R3P1",
  "gene_symbol": "MTRNR2L13",
  "term_label": "Unknown cellular component",
  "gene_name": "Humanin-like 13"
}